positive regulation of pheromone-dependent signal transduction involved in conjugation with cellular fusion [GO:0090028] (biological process) Relationships: is a type of regulation of pheromone-dependent signal transduction involved in conjugation with cellular fusion [GO:0010969]; is a type of positive regulation of signal transduction involved in conjugation with cellular fusion [GO:0060239]; positively regulates GO:0000750 Definition: Any process that increases the frequency, rate or extent of pheromone-dependent signal transduction during conjugation with cellular fusion, a signal transduction process resulting in the relay, amplification or dampening of a signal generated in response to pheromone exposure in organisms that undergo conjugation with cellular fusion. Sources: GOC:dph, GOC:tb